{
  "term_id": "GO:0015629",
  "gene_symbol": "SAMD14",
  "gene": "UniProtKB:Q8IZD0",
  "gene_name": "Sterile alpha motif domain-containing protein 14",
  "term_label": "actin cytoskeleton"
}